{
  "gene_symbol": "HTRA1",
  "term_id": "GO:0043065",
  "gene": "UniProtKB:Q92743",
  "term_label": "positive regulation of apoptotic process",
  "gene_name": "Serine protease HTRA1"
}